tubulin N-acetyltransferase activity [GO:0019799] (molecular function) Sources: EC:2.3.1.108 Relationships: is a type of protein-lysine-acetyltransferase activity [GO:0061733] Definition: Catalysis of the reaction: acetyl-CoA + (alpha-tubulin) L-lysine = CoA + (alpha-tubulin) N6-acetyl-L-lysine. In most organisms it acetylates L-lysine at position 40 of alpha- tubulin. Also known as: TAT activity, acetyl-CoA:alpha-tubulin-L-lysine 6-N-acetyltransferase activity, acetyl-CoA:alpha-tubulin-L-lysine N6-acetyltransferase activity, acetyl-CoA:alpha-tubulin-lysine N-acetyltransferase activity, alpha-tubulin N-acetyltransferase activity, alpha-tubulin acetylase activity, alpha-tubulin acetyltransferase activity, tubulin acetyltransferase activity